{
  "gene_symbol": "SGK1",
  "gene_name": "Serine_threonine-protein kinase Sgk1",
  "term_id": "GO:0005737",
  "gene": "UniProtKB:O00141",
  "term_label": "cytoplasm"
}